{
  "gene_symbol": "DUSP11",
  "term_label": "Unknown biological process",
  "gene": "UniProtKB:O75319",
  "gene_name": "RNA_RNP complex-1-interacting phosphatase",
  "term_id": "UNKNOWN:0002"
}